{
  "gene": "UniProtKB:Q9UF33",
  "gene_symbol": "EPHA6",
  "term_id": "GO:0005005",
  "gene_name": "Ephrin type-A receptor 6",
  "term_label": "transmembrane-ephrin receptor activity"
}